{
  "gene": "UniProtKB:Q9Y3T9",
  "gene_name": "Nucleolar complex protein 2 homolog",
  "term_label": "transcription corepressor activity",
  "term_id": "GO:0003714",
  "gene_symbol": "NOC2L"
}